negative regulation of hydrolase activity [GO:0051346] (BP) Definition: Any process that stops or reduces the rate of hydrolase activity, the catalysis of the hydrolysis of various bonds. Subtypes: negative regulation of peptidase activity [GO:0010466], GO:0010923, negative regulation of GTPase activity [GO:0034260], negative regulation of cyclic-nucleotide phosphodiesterase activity [GO:0051344], negative regulation of lipase activity [GO:0060192], negative regulation of all-trans-retinyl-ester hydrolase, 11-cis retinol forming activity [GO:0062003], negative regulation of beta-galactosidase activity [GO:1903770] Sources: GOC:ai Also known as: down regulation of hydrolase activity, down-regulation of hydrolase activity, downregulation of hydrolase activity, hydrolase inhibitor, inhibition of hydrolase activity Relationships: is a type of negative regulation of catalytic activity [GO:0043086]; is a type of GO:0051336; negatively regulates GO:0016787